{
  "gene_symbol": "PLLP",
  "gene": "UniProtKB:Q9Y342",
  "term_label": "myelination",
  "term_id": "GO:0042552",
  "gene_name": "Plasmolipin"
}